xylitol catabolic process [GO:0051160] (BP) Definition: The chemical reactions and pathways resulting in the breakdown of xylitol, a five-carbon sugar alcohol derived from xylose by reduction of the carbonyl group. Also known as: L-xylitol breakdown, L-xylitol catabolism, L-xylitol degradation Sources: GOC:ai Relationships: is a type of pentitol catabolic process [GO:0019527]; is a type of xylitol metabolic process [GO:0051164] Subtypes: xylitol catabolic process to D-xylulose 5-phosphate [GO:0019697] Note: Note that xylitol is a meso compound, thus there are no L or D-versions.